negative regulation of cell communication by chemical coupling [GO:0010653] (biological process) Sources: GOC:dph, GOC:kmv, GOC:tb Definition: Any process that decreases the frequency, rate or extent of cell communication via chemical coupling. Cell communication by chemical coupling is the process that mediates signaling interactions between one cell and another cell by the transfer of small, water-soluble molecules or metabolites between their adjacent cytoplasms via intercellular protein channels. Relationships: is_a GO:0010645; is a type of negative regulation of cell communication [GO:0010648]; RO_0002212 cell communication by chemical coupling [GO:0010643]